{
  "term_id": "UNKNOWN:0003",
  "gene": "UniProtKB:P17041",
  "term_label": "Unknown cellular component",
  "gene_name": "Zinc finger protein 32",
  "gene_symbol": "ZNF32"
}